{
  "gene_name": "Ribosomal RNA processing protein 1 homolog B",
  "gene_symbol": "RRP1B",
  "term_id": "GO:0006357",
  "term_label": "regulation of transcription by RNA polymerase II",
  "gene": "UniProtKB:Q14684"
}